{
  "gene": "UniProtKB:O14770",
  "gene_name": "Homeobox protein Meis2",
  "term_id": "GO:0007420",
  "term_label": "brain development",
  "gene_symbol": "MEIS2"
}